{
  "gene_name": "YTH domain-containing protein 1",
  "gene_symbol": "YTHDC1",
  "term_id": "GO:0000381",
  "gene": "UniProtKB:Q96MU7",
  "term_label": "regulation of alternative mRNA splicing, via spliceosome"
}